response to catechin [GO:1902168] (biological process) Definition: Any process that results in a change in state or activity of a cell or an organism (in terms of movement, secretion, enzyme production, gene expression, etc.) as a result of a catechin stimulus. References: PMID:23516620 Sources: GOC:TermGenie, GOC:rjd Relationships: is a type of response to phenylpropanoid [GO:0080184]; is a type of response to flavonoid [GO:1905395] Subtypes: cellular response to catechin [GO:1902169]